{
  "gene": "UniProtKB:Q8NGE3",
  "term_id": "GO:0005886",
  "gene_symbol": "OR10P1",
  "gene_name": "Olfactory receptor 10P1",
  "term_label": "plasma membrane"
}